{
  "gene": "UniProtKB:Q8WVZ9",
  "term_label": "regulation of Rac protein signal transduction",
  "term_id": "GO:0035020",
  "gene_symbol": "KBTBD7",
  "gene_name": "Kelch repeat and BTB domain-containing protein 7"
}